xylosylprotein 4-beta-galactosyltransferase activity [GO:0046525] (molecular function) Also known as: UDP-galactose:xylose galactosyltransferase activity, UDP-D-galactose:D-xylose galactosyltransferase activity, UDP-D-galactose:xylose galactosyltransferase activity, UDP-galactose:O-beta-D-xylosylprotein 4-beta-D-galactosyltransferase activity, UDPgalactose:O-beta-D-xylosylprotein 4-beta-D-galactosyltransferase activity, galactosyltransferase I activity, uridine diphosphogalactose-xylose galactosyltransferase activity Sources: EC:2.4.1.133 Definition: Catalysis of the reaction: UDP-galactose + O-beta-D-xylosylprotein = UDP + 4-beta-D-galactosyl-O-beta-D-xylosylprotein. Relationships: is a type of UDP-galactosyltransferase activity [GO:0035250]; is a type of catalytic activity, acting on a glycoprotein [GO:0140103]